{
  "term_id": "GO:0005923",
  "gene_name": "Multiple PDZ domain protein",
  "gene": "UniProtKB:O75970",
  "gene_symbol": "MPDZ",
  "term_label": "bicellular tight junction"
}